{
  "gene": "UniProtKB:Q68CQ4",
  "term_label": "small-subunit processome",
  "gene_symbol": "UTP25",
  "term_id": "GO:0032040",
  "gene_name": "U3 small nucleolar RNA-associated protein 25 homolog"
}